tricarboxylic acid catabolic process [GO:0072352] (biological process) Relationships: is a type of GO:0046395; is a type of GO:0072350 Sources: GOC:mah Definition: The chemical reactions and pathways resulting in the breakdown of dicarboxylic acids, any organic acid containing three carboxyl (-COOH) groups. Subtypes: GO:0019651, nicotianamine catabolic process [GO:0030419], 5,6,7,8-tetrahydrosarcinapterin catabolic process [GO:1901854] Also known as: tricarboxylate catabolic process, tricarboxylate catabolism, tricarboxylic acid breakdown, tricarboxylic acid catabolism, tricarboxylic acid degradation